{
  "gene_name": "Interferon alpha-inducible protein 27-like protein 2",
  "gene": "UniProtKB:Q9H2X8",
  "gene_symbol": "IFI27L2",
  "term_label": "molecular adaptor activity",
  "term_id": "GO:0060090"
}